{
  "gene_name": "Nucleolar protein 16",
  "term_label": "ribosomal large subunit biogenesis",
  "gene_symbol": "NOP16",
  "gene": "UniProtKB:Q9Y3C1",
  "term_id": "GO:0042273"
}